laminin-12 complex [GO:0043261] (cellular component) Relationships: is a type of laminin complex [GO:0043256] Definition: A laminin complex composed of alpha2, beta1 and gamma3 polypeptide chains. References: PMID:10842354 Sources: GOC:jl Also known as: laminin-213 complex